{
  "gene_name": "Aquaporin-5",
  "gene_symbol": "AQP5",
  "gene": "UniProtKB:P55064",
  "term_label": "water channel activity",
  "term_id": "GO:0015250"
}